{
  "term_id": "GO:0005886",
  "gene": "UniProtKB:Q9ULB1",
  "gene_symbol": "NRXN1",
  "gene_name": "Neurexin-1",
  "term_label": "plasma membrane"
}